endoribonuclease activity, cleaving miRNA-paired mRNA [GO:0090624] (molecular function) Definition: Catalysis of the endonucleolytic cleavage of the mRNA in a double-stranded RNA molecule formed by the base pairing of an mRNA with an miRNA. Relationships: is a type of RNA endonuclease activity producing 5'-phosphomonoesters, hydrolytic mechanism [GO:0016891]; is part of miRNA-mediated gene silencing by mRNA destabilization [GO:0035279] References: PMID:15260970, PMID:19239888 Sources: GOC:BHF, GOC:BHF_miRNA, GOC:rph